{
  "term_label": "external side of plasma membrane",
  "gene_symbol": "CEACAM21",
  "gene": "UniProtKB:Q3KPI0",
  "term_id": "GO:0009897",
  "gene_name": "Carcinoembryonic antigen-related cell adhesion molecule 21"
}